{
  "term_id": "GO:0016521",
  "gene": "UniProtKB:P18509",
  "gene_symbol": "ADCYAP1",
  "term_label": "pituitary adenylate cyclase activating polypeptide activity",
  "gene_name": "Pituitary adenylate cyclase-activating polypeptide"
}